{
  "gene_symbol": "AGAP1",
  "term_label": "GTPase activator activity",
  "gene_name": "Arf-GAP with GTPase, ANK repeat and PH domain-containing protein 1",
  "term_id": "GO:0005096",
  "gene": "UniProtKB:Q9UPQ3"
}